{
  "term_label": "U12-type spliceosomal complex",
  "term_id": "GO:0005689",
  "gene_name": "U11_U12 small nuclear ribonucleoprotein 25 kDa protein",
  "gene_symbol": "SNRNP25",
  "gene": "UniProtKB:Q9BV90"
}